{
  "gene": "UniProtKB:Q6NXP2",
  "term_label": "Unknown cellular component",
  "gene_symbol": "GARIN1A",
  "term_id": "UNKNOWN:0003",
  "gene_name": "Golgi-associated RAB2 interactor protein 1A"
}